galactitol metabolic process [GO:0019402] (biological process) Also known as: galactitol metabolism Sources: ISBN:0198506732 Relationships: is a type of hexitol metabolic process [GO:0006059] Subtypes: galactitol biosynthetic process [GO:0019403], galactitol catabolic process [GO:0019404] Definition: The chemical reactions and pathways involving galactitol, the hexitol derived by the reduction of the aldehyde group of either D- or L-galactose.